{
  "gene_symbol": "ZNF709",
  "gene_name": "Zinc finger protein 709",
  "gene": "UniProtKB:Q8N972",
  "term_label": "nucleus",
  "term_id": "GO:0005634"
}